{
  "gene": "UniProtKB:Q9H175",
  "gene_symbol": "CSRNP2",
  "term_id": "GO:0005634",
  "gene_name": "Cysteine_serine-rich nuclear protein 2",
  "term_label": "nucleus"
}